{
  "term_label": "proteolysis",
  "gene": "UniProtKB:P22891",
  "gene_symbol": "PROZ",
  "term_id": "GO:0006508",
  "gene_name": "Vitamin K-dependent protein Z"
}